{
  "gene_symbol": "UBN2",
  "term_id": "GO:0006325",
  "term_label": "chromatin organization",
  "gene": "UniProtKB:Q6ZU65",
  "gene_name": "Ubinuclein-2"
}